{
  "gene": "UniProtKB:Q9P242",
  "gene_symbol": "NYAP2",
  "term_id": "GO:0043491",
  "gene_name": "Neuronal tyrosine-phosphorylated phosphoinositide-3-kinase adapter 2",
  "term_label": "phosphatidylinositol 3-kinase/protein kinase B signal transduction"
}